regulation of Schwann cell migration [GO:1900147] (BP) Relationships: is a type of regulation of glial cell migration [GO:1903975]; regulates Schwann cell migration [GO:0036135] Subtypes: negative regulation of Schwann cell migration [GO:1900148], positive regulation of Schwann cell migration [GO:1900149], regulation of Schwann cell chemotaxis [GO:1904266] Sources: GOC:TermGenie, GOC:sjw Definition: Any process that modulates the frequency, rate or extent of Schwann cell migration.